{
  "gene_symbol": "HCN1",
  "term_label": "voltage-gated potassium channel activity",
  "gene": "UniProtKB:O60741",
  "term_id": "GO:0005249",
  "gene_name": "Potassium_sodium hyperpolarization-activated cyclic nucleotide-gated channel 1"
}